{
  "term_label": "DNA 5'-adenosine monophosphate hydrolase activity",
  "gene_symbol": "APTX",
  "gene_name": "Aprataxin",
  "term_id": "GO:0033699",
  "gene": "UniProtKB:Q7Z2E3"
}